{
  "gene": "UniProtKB:Q86TS9",
  "gene_name": "Large ribosomal subunit protein mL52",
  "term_id": "GO:0005762",
  "term_label": "mitochondrial large ribosomal subunit",
  "gene_symbol": "MRPL52"
}